{
  "gene": "UniProtKB:P32019",
  "gene_name": "Type II inositol 1,4,5-trisphosphate 5-phosphatase",
  "term_label": "cytosol",
  "gene_symbol": "INPP5B",
  "term_id": "GO:0005829"
}